{
  "gene": "UniProtKB:Q56UN5",
  "term_id": "UNKNOWN:0003",
  "gene_name": "Mitogen-activated protein kinase kinase kinase 19",
  "term_label": "Unknown cellular component",
  "gene_symbol": "MAP3K19"
}